{
  "term_id": "GO:0009880",
  "gene": "UniProtKB:A8K0S8",
  "gene_name": "Putative homeobox protein Meis3-like 2",
  "term_label": "embryonic pattern specification",
  "gene_symbol": "MEIS3P2"
}